hydroxyethylthiazole kinase activity [GO:0004417] (molecular function) Definition: Catalysis of the reaction: 5-(2-hydroxyethyl)-4-methylthiazole + ATP = 4-methyl-5-(2-phosphoethyl)-thiazole + ADP + 2 H+. Sources: EC:2.7.1.50, RHEA:24212 Relationships: is a type of kinase activity [GO:0016301]; is a type of GO:0016773 Also known as: 4-methyl-5-(beta-hydroxyethyl)thiazole kinase activity, ATP:4-methyl-5-(2-hydroxyethyl)thiazole 2-phosphotransferase activity, hydroxyethylthiazole kinase (phosphorylating)